{
  "gene_symbol": "TMEM255A",
  "term_id": "UNKNOWN:0002",
  "term_label": "Unknown biological process",
  "gene": "UniProtKB:Q5JRV8",
  "gene_name": "Transmembrane protein 255A"
}